{
  "gene_name": "Histone H2A.N",
  "gene_symbol": "H2BN1",
  "term_id": "UNKNOWN:0003",
  "gene": "UniProtKB:P0DW85",
  "term_label": "Unknown cellular component"
}